{
  "gene_name": "Multiple epidermal growth factor-like domains protein 10",
  "gene_symbol": "MEGF10",
  "term_id": "GO:0001891",
  "term_label": "phagocytic cup",
  "gene": "UniProtKB:Q96KG7"
}